{
  "gene": "UniProtKB:Q15293",
  "gene_symbol": "RCN1",
  "gene_name": "Reticulocalbin-1",
  "term_id": "GO:0005783",
  "term_label": "endoplasmic reticulum"
}